{
  "gene_name": "Zinc finger protein 285",
  "term_label": "Unknown molecular function",
  "term_id": "UNKNOWN:0001",
  "gene": "UniProtKB:Q96NJ3",
  "gene_symbol": "ZNF285"
}